monoatomic anion:monoatomic cation symporter activity [GO:0015296] (molecular function) Relationships: is a type of monoatomic anion transmembrane transporter activity [GO:0008509]; is a type of solute:monoatomic cation symporter activity [GO:0015294] Definition: Enables the transfer of a solute or solutes from one side of a membrane to the other according to the reaction: anion(out) + cation(out) = anion(in) + cation(in). Subtypes: monoatomic anion:sodium symporter activity [GO:0015373], chloride:monoatomic cation symporter activity [GO:0015377] Also known as: anion:cation symporter activity Sources: TC:2.A.1.14.-